vitamin D binding [GO:0005499] (MF) Relationships: is a type of steroid binding [GO:0005496]; is a type of vitamin binding [GO:0019842] Also known as: calciferol binding, cholecalciferol binding, ergocalciferol binding Definition: Binding to vitamin D, any of a group of related, fat-soluble compounds that are derived from delta-5,7 steroids and play a central role in calcium metabolism. Specific forms of vitamin D include calciferol (ergocalciferol; vitamin D2) and cholecalciferol (calciol; vitamin D3). Subtypes: D3 vitamins binding [GO:1902271] Sources: GOC:mah, ISBN:0471331309